regulation of microtubule cytoskeleton organization [GO:0070507] (biological process) Definition: Any process that modulates the frequency, rate or extent of the formation, arrangement of constituent parts, or disassembly of cytoskeletal structures comprising microtubules and their associated proteins. Sources: GOC:mah Also known as: regulation of microtubule cytoskeleton organisation, regulation of microtubule dynamics Relationships: is a type of regulation of microtubule-based process [GO:0032886]; is a type of regulation of cytoskeleton organization [GO:0051493]; regulates microtubule cytoskeleton organization [GO:0000226] Subtypes: regulation of microtubule polymerization or depolymerization [GO:0031110], Wnt signaling pathway, regulating spindle positioning [GO:0060069], regulation of spindle organization [GO:0090224], regulation of microtubule anchoring at centrosome [GO:0150101], GO:2000694